{
  "gene_name": "Peptidylprolyl isomerase domain and WD repeat-containing protein 1",
  "gene": "UniProtKB:Q96BP3",
  "term_id": "UNKNOWN:0003",
  "term_label": "Unknown cellular component",
  "gene_symbol": "PPWD1"
}